CO-methylating acetyl-CoA synthase activity [GO:0043884] (molecular function) References: PMID:1748656 Sources: EC:2.3.1.169 Definition: Catalysis of the reaction: acetyl-CoA + corrinoid protein = CO + methylcorrinoid protein + CoA. Also known as: acetyl-CoA synthase activity, CO-methylating acetyl-coenzyme A synthase activity, acetyl-CoA:corrinoid protein O-acetyltransferase activity, ACS Relationships: is_a acyltransferase activity, transferring groups other than amino-acyl groups [GO:0016747]